acylglycerol kinase activity [GO:0047620] (molecular function) Also known as: ATP:acylglycerol 3-phosphotransferase activity, MGK, monoacylglycerol kinase (phosphorylating), monoacylglycerol kinase activity, monoglyceride kinase activity, monoglyceride phosphokinase activity, sn-2-monoacylglycerol kinase activity Relationships: is a type of kinase activity [GO:0016301]; is a type of phosphotransferase activity, alcohol group as acceptor [GO:0016773] Sources: EC:2.7.1.94, MetaCyc:ACYLGLYCEROL-KINASE-RXN Definition: Catalysis of the reaction: ATP + acylglycerol = ADP + acyl-sn-glycerol 3-phosphate.